{
  "gene": "UniProtKB:Q9NYG5",
  "gene_name": "Anaphase-promoting complex subunit 11",
  "gene_symbol": "ANAPC11",
  "term_id": "GO:0006511",
  "term_label": "ubiquitin-dependent protein catabolic process"
}